ent-cassa-12,15-diene synthase activity [GO:0034277] (molecular function) Relationships: is a type of GO:0016838 Also known as: ent-copalyl-diphosphate diphosphate-lyase (ent-cassa-12,15-diene-forming) activity Definition: Catalysis of the reaction: ent-copalyl diphosphate = ent-cassa-12,15-diene + diphosphate. Sources: EC:4.2.3.28, RHEA:25532